{
  "gene_symbol": "HRCT1",
  "term_id": "UNKNOWN:0003",
  "gene": "UniProtKB:Q6UXD1",
  "term_label": "Unknown cellular component",
  "gene_name": "Histidine-rich carboxyl terminus protein 1"
}